{
  "gene": "UniProtKB:B1ANS9",
  "term_id": "UNKNOWN:0002",
  "term_label": "Unknown biological process",
  "gene_symbol": "WDR64",
  "gene_name": "WD repeat-containing protein 64"
}